{
  "gene_symbol": "SOX14",
  "term_id": "GO:0045944",
  "gene_name": "Transcription factor SOX-14",
  "gene": "UniProtKB:O95416",
  "term_label": "positive regulation of transcription by RNA polymerase II"
}